{
  "gene_symbol": "DUSP1",
  "term_label": "phosphoprotein phosphatase activity",
  "term_id": "GO:0004721",
  "gene": "UniProtKB:P28562",
  "gene_name": "Dual specificity protein phosphatase 1"
}